iron import into the mitochondrion [GO:0048250] (biological process) Relationships: is a type of GO:0034755 References: PMID:12006577 Sources: GOC:jid Definition: The process in which iron is transported from the cytosol into the mitochondrial matrix. Also known as: mitochondrial iron cation transmembrane transport, mitochondrial iron transport, mitochondrial iron ion transmembrane transport, mitochondrial iron ion transport